{
  "gene_name": "STARD3 N-terminal-like protein",
  "term_id": "GO:0140284",
  "gene_symbol": "STARD3NL",
  "gene": "UniProtKB:O95772",
  "term_label": "endoplasmic reticulum-endosome membrane contact site"
}